negative regulation of oskar mRNA translation [GO:0007319] (biological process) Relationships: is a type of negative regulation of translation [GO:0017148]; is a type of regulation of oskar mRNA translation [GO:0046011] Sources: GOC:ems Definition: Any process that stops, prevents or reduces the rate that oskar mRNAs are effectively translated into protein. Also known as: down regulation of oskar mRNA translation, down-regulation of oskar mRNA translation, downregulation of oskar mRNA translation, inhibition of oskar mRNA translation